{
  "gene_name": "Bone morphogenetic protein receptor type-1B",
  "gene_symbol": "BMPR1B",
  "term_label": "BMP signaling pathway",
  "term_id": "GO:0030509",
  "gene": "UniProtKB:O00238"
}